glycerol-3-phosphate shuttle [GO:0006127] (BP) Definition: The process of transferring reducing equivalents from NADH in the cytosol into the mitochondria via glycerol-3-phosphate. Cytosolic glycerol-3-phosphate dehydrogenase uses NADH to convert dihydroxyacetone phosphate (DHAP) to glycerol-3-phosphate (G3P) in the cytosol; G3P then diffuses into the mitochondria where mitochondrial glycerol-3-phosphate dehydrogenase uses FAD to convert G3P back to DHAP; the electrons on the reduced FADH2 are then available for use in the electron transport chain, and DHAP returns to the cytosol to complete the cycle. References: PMID:16368075 Sources: GOC:sjm Also known as: glycerol phosphate shuttle, glycerophosphate shuttle Relationships: is a type of NAD+ metabolic process [GO:0019674]; has part glycerol-3-phosphate dehydrogenase (quinone) activity [GO:0004368]; has part glycerol-3-phosphate dehydrogenase (NAD+) activity [GO:0141152]